cardiac right atrium morphogenesis [GO:0003213] (biological process) Sources: GOC:mtg_heart Definition: The process in which the right cardiac atrium is generated and organized. Relationships: is a type of GO:0003209